{
  "term_label": "heterochromatin",
  "gene": "UniProtKB:Q14781",
  "gene_name": "Chromobox protein homolog 2",
  "gene_symbol": "CBX2",
  "term_id": "GO:0000792"
}